{
  "gene_symbol": "HMCN1",
  "gene": "UniProtKB:Q96RW7",
  "gene_name": "Hemicentin-1",
  "term_id": "GO:0007156",
  "term_label": "homophilic cell-cell adhesion"
}